{
  "gene_name": "Endoplasmic reticulum transmembrane helix translocase",
  "term_id": "GO:0140567",
  "gene": "UniProtKB:Q9HD20",
  "gene_symbol": "ATP13A1",
  "term_label": "membrane protein dislocase activity"
}